{
  "gene_name": "Ribosyldihydronicotinamide dehydrogenase [quinone]",
  "gene_symbol": "NQO2",
  "term_label": "NAD(P)H dehydrogenase (quinone) activity",
  "gene": "UniProtKB:P16083",
  "term_id": "GO:0003955"
}